neuromast hair cell morphogenesis [GO:0035678] (biological process) Definition: The change in form (cell shape and size) that occurs when a neuromast hair cell progresses from its initial formation to its mature state. A neuromast hair cell is a hair cell that acts as a sensory receptor of the neuromast; it is morphologically polarized as a result of the relative position of the single kinocilium and the clusters of stereocilia on its apical surface. Sources: CL:0000856 Relationships: is a type of cell morphogenesis involved in neuron differentiation [GO:0048667]; is part of GO:0035675 Subtypes: anterior lateral line neuromast hair cell morphogenesis [GO:0035679], GO:0035680